{
  "term_label": "structural constituent of ribosome",
  "gene_name": "Large ribosomal subunit protein mL49",
  "gene": "UniProtKB:Q13405",
  "gene_symbol": "MRPL49",
  "term_id": "GO:0003735"
}